5-(3,4-diacetoxybut-1-ynyl)-2,2'-bithiophene deacetylase activity [GO:0047377] (molecular function) Definition: Catalysis of the reaction: 5-(3,4-diacetoxybut-1-ynyl)-2,2'-bithiophene + H2O = 5-(3-hydroxy-4-acetoxybut-1-ynyl)-2,2'-bithiophene + acetate + H+. Sources: EC:3.1.1.66, RHEA:16313 Relationships: is_a deacetylase activity [GO:0019213]; is a type of carboxylic ester hydrolase activity [GO:0052689] Also known as: 3,4-diacetoxybutinylbithiophene:4-acetate esterase activity, 5-(3,4-diacetoxybut-1-ynyl)-2,2'-bithiophene acetylhydrolase activity, diacetoxybutynylbithiophene acetate esterase activity